cell wall pectin biosynthetic process [GO:0052325] (biological process) Definition: The chemical reactions and pathways resulting in the formation of pectin, a polymer containing a backbone of alpha-1,4-linked D-galacturonic acid residues, as part of the organization and biogenesis of the cell wall. Sources: GOC:ai Also known as: cell wall pectin biosynthesis, pectin biosynthesis during cell wall organization and biogenesis Relationships: is a type of GO:0045489; is a type of cell wall pectin metabolic process [GO:0052546]; is_a cell wall polysaccharide biosynthetic process [GO:0070592]; is part of plant-type cell wall biogenesis [GO:0009832] Subtypes: homogalacturonan biosynthetic process [GO:0010289], rhamnogalacturonan II biosynthetic process [GO:0010306]